{
  "term_id": "GO:0001517",
  "gene_symbol": "CHST7",
  "gene_name": "Carbohydrate sulfotransferase 7",
  "gene": "UniProtKB:Q9NS84",
  "term_label": "N-acetylglucosamine 6-O-sulfotransferase activity"
}